{
  "term_id": "GO:0005922",
  "gene": "UniProtKB:P35212",
  "term_label": "connexin complex",
  "gene_symbol": "GJA4",
  "gene_name": "Gap junction alpha-4 protein"
}